{
  "gene_name": "E3 ubiquitin-protein ligase RBX1",
  "term_id": "GO:0061630",
  "gene_symbol": "RBX1",
  "term_label": "ubiquitin protein ligase activity",
  "gene": "UniProtKB:P62877"
}